{
  "gene_name": "Solute carrier family 12 member 8",
  "term_label": "chloride ion homeostasis",
  "term_id": "GO:0055064",
  "gene_symbol": "SLC12A8",
  "gene": "UniProtKB:A0AV02"
}